{
  "gene_name": "Nidogen-1",
  "term_label": "Unknown cellular component",
  "gene_symbol": "NID1",
  "gene": "UniProtKB:P14543",
  "term_id": "UNKNOWN:0003"
}